regulation of B cell antigen processing and presentation [GO:0002622] (biological process) Subtypes: negative regulation of B cell antigen processing and presentation [GO:0002623], positive regulation of B cell antigen processing and presentation [GO:0002624] Also known as: regulation of B lymphocyte antigen processing and presentation, regulation of B-cell antigen processing and presentation, regulation of B-lymphocyte antigen processing and presentation Relationships: is a type of GO:0002577; is a type of regulation of B cell mediated immunity [GO:0002712]; regulates B cell antigen processing and presentation [GO:0002450] Definition: Any process that modulates the frequency, rate, or extent of B cell antigen processing and presentation. Sources: GOC:add